{
  "gene": "UniProtKB:O75909",
  "gene_name": "Cyclin-K",
  "term_label": "positive regulation of transcription by RNA polymerase II",
  "term_id": "GO:0045944",
  "gene_symbol": "CCNK"
}